{
  "term_id": "UNKNOWN:0002",
  "term_label": "Unknown biological process",
  "gene_symbol": "RDH14",
  "gene": "UniProtKB:Q9HBH5",
  "gene_name": "Retinol dehydrogenase 14"
}